{
  "gene": "UniProtKB:O00443",
  "gene_name": "Phosphatidylinositol 4-phosphate 3-kinase C2 domain-containing subunit alpha",
  "term_label": "plasma membrane",
  "gene_symbol": "PIK3C2A",
  "term_id": "GO:0005886"
}